{
  "gene_name": "Serine_threonine-protein phosphatase 2A 56 kDa regulatory subunit delta isoform",
  "gene_symbol": "PPP2R5D",
  "gene": "UniProtKB:Q14738",
  "term_label": "protein phosphatase activator activity",
  "term_id": "GO:0072542"
}